{
  "gene_symbol": "HOMER1",
  "gene_name": "Homer protein homolog 1",
  "term_id": "GO:0007216",
  "gene": "UniProtKB:Q86YM7",
  "term_label": "G protein-coupled glutamate receptor signaling pathway"
}